{
  "gene_name": "Embigin",
  "gene_symbol": "EMB",
  "term_label": "cell-cell adhesion mediator activity",
  "term_id": "GO:0098632",
  "gene": "UniProtKB:Q6PCB8"
}